{
  "term_id": "UNKNOWN:0003",
  "gene": "UniProtKB:Q96RT1",
  "gene_name": "Erbin",
  "term_label": "Unknown cellular component",
  "gene_symbol": "ERBIN"
}